TDP biosynthetic process [GO:0006232] (biological process) Definition: The chemical reactions and pathways resulting in the formation of TDP, ribosylthymine diphosphate. Sources: ISBN:0198506732 Relationships: is a type of GO:0009194; is a type of GO:0009220; is a type of TDP metabolic process [GO:0046043] Also known as: TDP anabolism, TDP biosynthesis, TDP formation, TDP synthesis